{
  "gene_symbol": "KIF1A",
  "term_label": "axon",
  "term_id": "GO:0030424",
  "gene": "UniProtKB:Q12756",
  "gene_name": "Kinesin-like protein KIF1A"
}